{
  "gene_name": "Methionine-R-sulfoxide reductase B3",
  "gene_symbol": "MSRB3",
  "term_label": "Unknown biological process",
  "gene": "UniProtKB:Q8IXL7",
  "term_id": "UNKNOWN:0002"
}